styrene-oxide isomerase activity [GO:0018846] (molecular function) Sources: EC:5.3.99.7, RHEA:21604 Relationships: is a type of intramolecular oxidoreductase activity [GO:0016860] Definition: Catalysis of the reaction: styrene oxide = phenylacetaldehyde. Also known as: styrene oxide isomerase activity, SOI activity, styrene-oxide isomerase (epoxide-cleaving)